{
  "gene_symbol": "MAGEL2",
  "term_id": "GO:0000122",
  "term_label": "negative regulation of transcription by RNA polymerase II",
  "gene_name": "MAGE-like protein 2",
  "gene": "UniProtKB:Q9UJ55"
}